{
  "gene": "UniProtKB:Q9NQS7",
  "gene_name": "Inner centromere protein",
  "term_label": "mitotic cytokinesis",
  "gene_symbol": "INCENP",
  "term_id": "GO:0000281"
}